biliberdin reductase (NADH) activity [GO:0106276] (MF) Definition: Catalysis of the reaction: bilirubin IXalpha + NAD+ = biliverdin IXalpha + NADH+ H+. Sources: RHEA:15797 Also known as: biliberdin reductase (NAD+) activity Relationships: is_a biliverdin reductase [NAD(P)H] activity [GO:0004074]